{
  "gene_name": "Cation-dependent mannose-6-phosphate receptor",
  "gene_symbol": "M6PR",
  "term_label": "trans-Golgi network",
  "term_id": "GO:0005802",
  "gene": "UniProtKB:P20645"
}